{
  "term_label": "RNA binding",
  "gene_symbol": "SEC63",
  "gene_name": "Translocation protein SEC63 homolog",
  "gene": "UniProtKB:Q9UGP8",
  "term_id": "GO:0003723"
}